{
  "gene": "UniProtKB:P00747",
  "gene_symbol": "PLG",
  "term_id": "GO:0005102",
  "gene_name": "Plasminogen",
  "term_label": "signaling receptor binding"
}